cytoplasmic side of membrane [GO:0098562] (cellular component) Definition: The side of a membrane that faces the cytoplasm. Sources: GOC:dos Relationships: is a type of side of membrane [GO:0098552] Subtypes: GO:0009898, cytoplasmic side of endosome membrane [GO:0010009], GO:0032473, cytoplasmic side of transport vesicle membrane [GO:0098539], cytoplasmic side of Golgi membrane [GO:0098548], cytoplasmic side of endoplasmic reticulum membrane [GO:0098554], cytoplasmic side of lysosomal membrane [GO:0098574], cytoplasmic side of cis-Golgi network membrane [GO:0140179], cytoplasmic side of cis-Golgi cisternae membrane [GO:0160278], cytoplasmic side of medial-Golgi cisterna membrane [GO:0160279], GO:0160281, cytoplasmic side of trans-Golgi cisterna membrane [GO:0160288]